folic acid catabolic process [GO:0046657] (biological process) Also known as: folate catabolic process, folate catabolism, folic acid breakdown, folic acid catabolism, folic acid degradation, vitamin B9 catabolic process, vitamin B9 catabolism, vitamin M catabolic process, vitamin M catabolism Definition: The chemical reactions and pathways resulting in the breakdown of folic acid, pteroylglutamic acid. Sources: GOC:ai Relationships: is a type of folic acid-containing compound catabolic process [GO:0009397]; is a type of water-soluble vitamin catabolic process [GO:0042365]; is a type of dicarboxylic acid catabolic process [GO:0043649]; is a type of folic acid metabolic process [GO:0046655]